interleukin-20 binding [GO:0042015] (molecular function) Relationships: is a type of cytokine binding [GO:0019955] Sources: GOC:jl Definition: Binding to interleukin-20. Also known as: IL-20 binding